negative regulation of adaptive immune effector response [GO:1905678] (biological process) Definition: Any process that stops, prevents or reduces the frequency, rate or extent of adaptive immune effector response. Relationships: is a type of negative regulation of adaptive immune response [GO:0002820]; is a type of regulation of adaptive immune effector response [GO:1905677]; negatively regulates adaptive immune effector response [GO:0090718] Sources: GOC:TermGenie, GO_REF:0000058, ISBN:9781405196833 Also known as: down regulation of adaptive immune effector response, down-regulation of adaptive immune effector response, downregulation of adaptive immune effector response, inhibition of adaptive immune effector response